detection of oxygen [GO:0003032] (biological process) Definition: The series of events in which an oxygen stimulus is received by a cell and converted into a molecular signal. Relationships: is a type of GO:0009593; is a type of response to oxygen levels [GO:0070482] Subtypes: detection of hypoxia [GO:0070483] Sources: GOC:mtg_cardio